actin filament bundle distribution [GO:0070650] (biological process) Relationships: is a type of actin filament bundle organization [GO:0061572] Subtypes: actin filament bundle retrograde transport [GO:0061573], actin filament bundle convergence [GO:0090426] Definition: Any cellular process that establishes the spatial arrangement of actin filament bundles within the cell. Sources: GOC:mah